2-phytyl-1,4-naphthoquinone methyltransferase activity [GO:0052624] (molecular function) Definition: Catalysis of the reaction: demethylphylloquinol + S-adenosyl-L-methionine = H+ + phylloquinol + S-adenosyl-L-homocysteine. Relationships: is a type of C-methyltransferase activity [GO:0008169]; is a type of O-methyltransferase activity [GO:0008171] Also known as: SA methyltransferase activity, salicylate methyltransferase activity, salicylic acid methyltransferase activity, S-adenosyl-L-methionine:2-phytyl-1,4-naphthoquinone methyltransferase activity, S-adenosyl-L-methionine:demethylphylloquinone methyltransferase activity, S-adenosyl-L-methionine:salicylate carboxyl methyltransferase activity, demethylphylloquinone methyltransferase activity References: PMID:14617060 Sources: RHEA:40551